{
  "gene": "UniProtKB:P78504",
  "term_id": "UNKNOWN:0002",
  "term_label": "Unknown biological process",
  "gene_name": "Protein jagged-1",
  "gene_symbol": "JAG1"
}